{
  "gene_symbol": "FOXO3B",
  "gene": "UniProtKB:A0A2Z4LIS9",
  "term_label": "mitochondrial matrix",
  "term_id": "GO:0005759",
  "gene_name": "Forkhead box protein O3B"
}